positive regulation of ribosomal small subunit export from nucleus [GO:2000208] (biological process) Relationships: is_a positive regulation of ribosomal subunit export from nucleus [GO:2000202]; is a type of regulation of ribosomal small subunit export from nucleus [GO:2000206]; positively regulates ribosomal small subunit export from nucleus [GO:0000056] Also known as: positive regulation of ribosomal small subunit export from cell nucleus, positive regulation of ribosomal small subunit export out of nucleus, positive regulation of ribosomal small subunit transport from nucleus to cytoplasm, positive regulation of ribosomal small subunit-nucleus export, positive regulation of 30S ribosomal subunit export from nucleus, positive regulation of 40S ribosomal subunit export from nucleus Definition: Any process that activates or increases the frequency, rate or extent of ribosomal small subunit export from nucleus. Sources: GOC:mah